negative regulation of pre-miRNA processing [GO:2000632] (biological process) Relationships: is_a negative regulation of miRNA processing [GO:1903799]; is a type of GO:2000631; RO_0002212 pre-miRNA processing [GO:0031054] Definition: Any process that stops, prevents or reduces the frequency, rate or extent of pre-microRNA processing. Sources: GOC:dph, GOC:sl Also known as: negative regulation of miRNA maturation, negative regulation of pre-microRNA processing